{
  "term_id": "GO:0005768",
  "gene": "UniProtKB:Q9Y328",
  "gene_name": "Neuronal vesicle trafficking-associated protein 2",
  "term_label": "endosome",
  "gene_symbol": "NSG2"
}